{
  "gene": "UniProtKB:A2A3N6",
  "gene_name": "Putative PIP5K1A and PSMD4-like protein",
  "term_id": "GO:0046854",
  "gene_symbol": "PIPSL",
  "term_label": "phosphatidylinositol phosphate biosynthetic process"
}